{
  "gene_symbol": "C17orf114",
  "gene": "UniProtKB:A0A1B0GUV1",
  "term_label": "Unknown molecular function",
  "term_id": "UNKNOWN:0001",
  "gene_name": "Uncharacterized protein C17orf114"
}